trachea submucosa development [GO:0061152] (biological process) Relationships: is a type of anatomical structure development [GO:0048856]; is part of trachea development [GO:0060438] Definition: The progression of the trachea submucosa over time from its formation to the mature structure. The trachea submucosa is made up of the glands and elastic tissue that lie under the mucosa in the trachea. Sources: GOC:dph, GOC:yaf